{
  "gene": "UniProtKB:P30926",
  "term_id": "GO:0051899",
  "term_label": "membrane depolarization",
  "gene_name": "Neuronal acetylcholine receptor subunit beta-4",
  "gene_symbol": "CHRNB4"
}